{
  "gene_name": "eIF5-mimic protein 2",
  "gene_symbol": "BZW1",
  "term_label": "Unknown biological process",
  "term_id": "UNKNOWN:0002",
  "gene": "UniProtKB:Q7L1Q6"
}